heptaprenyl diphosphate synthase activity [GO:0000010] (molecular function) References: PMID:9708911 Sources: RHEA:27794 Definition: Catalysis of the reaction: (2E,6E)-farnesyl diphosphate + 4 isopentenyl diphosphate = 4 diphosphate + all-trans-heptaprenyl diphosphate. Relationships: is a type of prenyl diphosphate synthase activity [GO:0120531] Also known as: all-trans-heptaprenyl-diphosphate synthase activity, trans-hexaprenyltranstransferase activity, HepPP synthase activity, heptaprenyl pyrophosphate synthase activity, heptaprenyl pyrophosphate synthetase activity